{
  "term_id": "UNKNOWN:0002",
  "gene_name": "N-acetylneuraminate 9-O-acetyltransferase",
  "gene_symbol": "CASD1",
  "gene": "UniProtKB:Q96PB1",
  "term_label": "Unknown biological process"
}